{
  "gene": "UniProtKB:P43363",
  "gene_name": "Melanoma-associated antigen 10",
  "gene_symbol": "MAGEA10",
  "term_label": "nucleus",
  "term_id": "GO:0005634"
}